{
  "gene": "UniProtKB:Q86T20",
  "gene_symbol": "SMIM29",
  "term_id": "UNKNOWN:0002",
  "gene_name": "Small integral membrane protein 29",
  "term_label": "Unknown biological process"
}